exocytosis [GO:0006887] (biological process) References: PMID:22323285 Sources: GOC:mah, ISBN:0716731363 Subtypes: constitutive secretory pathway [GO:0045054], regulated exocytosis [GO:0045055], GO:0098967, GO:0160192, exosomal secretion [GO:1990182] Regulation: regulated by regulation of exocytosis [GO:0017157]; negatively regulated by GO:0045920; positively regulated by positive regulation of exocytosis [GO:0045921] Relationships: is a type of vesicle-mediated transport [GO:0016192]; is_a secretion by cell [GO:0032940]; has part vesicle fusion to plasma membrane [GO:0099500] Definition: A process of secretion by a cell that results in the release of intracellular molecules (e.g. hormones, matrix proteins) contained within a membrane-bounded vesicle. Exocytosis can occur either by full fusion, when the vesicle collapses into the plasma membrane, or by a kiss-and-run mechanism that involves the formation of a transient contact, a pore, between a granule (for example of chromaffin cells) and the plasma membrane. The latter process most of the time leads to only partial secretion of the granule content. Exocytosis begins with steps that prepare vesicles for fusion with the membrane (tethering and docking) and ends when molecules are secreted from the cell. Also known as: vesicle exocytosis, nonselective vesicle exocytosis